negative regulation of astrocyte chemotaxis [GO:2000459] (biological process) Relationships: is a type of negative regulation of chemotaxis [GO:0050922]; is a type of negative regulation of glial cell migration [GO:1903976]; is a type of regulation of astrocyte chemotaxis [GO:2000458]; negatively regulates GO:0035700 Definition: Any process that stops, prevents or reduces the frequency, rate or extent of astrocyte chemotaxis. Sources: GOC:obol